{
  "term_label": "plasma membrane",
  "gene_symbol": "RASGRP2",
  "gene": "UniProtKB:Q7LDG7",
  "term_id": "GO:0005886",
  "gene_name": "RAS guanyl-releasing protein 2"
}